{
  "gene_symbol": "FGF17",
  "term_label": "regulation of cell migration",
  "term_id": "GO:0030334",
  "gene_name": "Fibroblast growth factor 17",
  "gene": "UniProtKB:O60258"
}